{
  "gene": "UniProtKB:P16871",
  "gene_symbol": "IL7R",
  "term_label": "positive regulation of receptor signaling pathway via JAK-STAT",
  "gene_name": "Interleukin-7 receptor subunit alpha",
  "term_id": "GO:0046427"
}